{
  "term_id": "GO:0003682",
  "gene": "UniProtKB:P54253",
  "gene_symbol": "ATXN1",
  "term_label": "chromatin binding",
  "gene_name": "Ataxin-1"
}